{
  "gene_name": "C-C motif chemokine 5",
  "gene_symbol": "CCL5",
  "gene": "UniProtKB:P13501",
  "term_id": "GO:0061844",
  "term_label": "antimicrobial humoral immune response mediated by antimicrobial peptide"
}